{
  "gene": "UniProtKB:Q8IV76",
  "gene_name": "Circadian clock protein PASD1",
  "term_label": "regulation of transcription by RNA polymerase II",
  "gene_symbol": "PASD1",
  "term_id": "GO:0006357"
}